{
  "term_id": "GO:0001525",
  "gene_name": "G-protein coupled receptor 15",
  "term_label": "angiogenesis",
  "gene_symbol": "GPR15",
  "gene": "UniProtKB:P49685"
}